regulation of maltose transport [GO:1902343] (biological process) Relationships: is a type of regulation of transport [GO:0051049]; regulates maltose transport [GO:0015768] References: PMID:23770568 Sources: GOC:TermGenie, GOC:dph Subtypes: negative regulation of maltose transport [GO:1902344], positive regulation of maltose transport [GO:1902345] Definition: Any process that modulates the frequency, rate or extent of maltose transport.